{
  "gene_name": "T-cell leukemia_lymphoma protein 1A",
  "term_label": "nucleus",
  "gene_symbol": "TCL1A",
  "term_id": "GO:0005634",
  "gene": "UniProtKB:P56279"
}